{
  "term_label": "Unknown cellular component",
  "term_id": "UNKNOWN:0003",
  "gene_symbol": "ZNF85",
  "gene_name": "Zinc finger protein 85",
  "gene": "UniProtKB:Q03923"
}